apoptotic process involved in morphogenesis [GO:0060561] (biological process) Definition: Any apoptotic process that contributes to the shaping of an anatomical structure. Also known as: apoptosis involved in morphogenesis, apoptosis involved in development, morphogenetic apoptosis Relationships: is a type of apoptotic process involved in development [GO:1902742]; is part of anatomical structure morphogenesis [GO:0009653] Regulation: regulated by regulation of apoptotic process involved in morphogenesis [GO:1902337]; negatively regulated by negative regulation of apoptotic process involved in morphogenesis [GO:1902338]; positively regulated by positive regulation of apoptotic process involved in morphogenesis [GO:1902339] Subtypes: GO:0003278, apoptotic process involved in mammary gland involution [GO:0060057], apoptotic process involved in tube lumen cavitation [GO:0060609], clearance of cells from fusion plate by apoptotic process [GO:0060885], mesenchymal cell apoptotic process involved in nephron morphogenesis [GO:1901145], apoptotic process involved in blood vessel morphogenesis [GO:1902262], apoptotic process involved in embryonic digit morphogenesis [GO:1902263], epithelial cell apoptotic process involved in palatal shelf morphogenesis [GO:1990134] Sources: GOC:dph, GOC:mtg_apoptosis